interleukin-19 production [GO:0032622] (biological process) Relationships: is a type of cytokine production [GO:0001816] Sources: GOC:mah Definition: The appearance of interleukin-19 due to biosynthesis or secretion following a cellular stimulus, resulting in an increase in its intracellular or extracellular levels. Also known as: IL-19 production, IL-19 secretion, ZMDA1 secretion, interleukin-19 biosynthetic process, interleukin-19 secretion Regulation: regulated by regulation of interleukin-19 production [GO:0032662]; negatively regulated by negative regulation of interleukin-19 production [GO:0032702]; positively regulated by positive regulation of interleukin-19 production [GO:0032742]